{
  "term_id": "UNKNOWN:0002",
  "gene_name": "Ectonucleotide pyrophosphatase_phosphodiesterase family member 5",
  "gene_symbol": "ENPP5",
  "term_label": "Unknown biological process",
  "gene": "UniProtKB:Q9UJA9"
}